{
  "gene_name": "Zinc finger and SCAN domain-containing protein 25",
  "term_id": "GO:0000981",
  "term_label": "DNA-binding transcription factor activity, RNA polymerase II-specific",
  "gene": "UniProtKB:Q6NSZ9",
  "gene_symbol": "ZSCAN25"
}